{
  "gene": "UniProtKB:P54289",
  "gene_name": "Voltage-dependent calcium channel subunit alpha-2_delta-1",
  "gene_symbol": "CACNA2D1",
  "term_id": "GO:1990454",
  "term_label": "L-type voltage-gated calcium channel complex"
}